{
  "term_label": "axon",
  "term_id": "GO:0030424",
  "gene_symbol": "ROR2",
  "gene": "UniProtKB:Q01974",
  "gene_name": "Tyrosine-protein kinase transmembrane receptor ROR2"
}